{
  "term_label": "nucleus",
  "gene_symbol": "UBE2N",
  "gene_name": "Ubiquitin-conjugating enzyme E2 N",
  "term_id": "GO:0005634",
  "gene": "UniProtKB:P61088"
}